regulation of G protein-coupled receptor signaling pathway [GO:0008277] (biological process) Definition: Any process that modulates the frequency, rate or extent of G protein-coupled receptor signaling pathway. Sources: GOC:go_curators Also known as: regulation of G protein coupled receptor protein signaling pathway, regulation of G protein coupled receptor protein signalling pathway, regulation of G-protein coupled receptor protein signaling pathway, regulation of G-protein coupled receptor protein signalling pathway, regulation of G-protein-coupled receptor protein signalling pathway, regulation of GPCR protein signaling pathway, regulation of GPCR protein signalling pathway Relationships: is a type of regulation of signal transduction [GO:0009966]; regulates GO:0007186 Subtypes: GO:0022400, cross-receptor inhibition within G protein-coupled receptor heterodimer [GO:0038041], protein kinase C deactivation [GO:0042313], negative regulation of G protein-coupled receptor signaling pathway [GO:0045744], positive regulation of G protein-coupled receptor signaling pathway [GO:0045745], regulation of dopamine receptor signaling pathway [GO:0060159], regulation of adenosine receptor signaling pathway [GO:0060167], GO:0070099, regulation of thrombin-activated receptor signaling pathway [GO:0070494], regulation of adenylate cyclase-inhibiting adrenergic receptor signaling pathway [GO:0071877], GO:0106070, regulation of angiotensin-activated signaling pathway [GO:0110061], GO:1900736, GO:1904020, GO:2000124, regulation of octopamine or tyramine signaling pathway [GO:2000125], regulation of opioid receptor signaling pathway [GO:2000474]